negative regulation of L-tyrosine import across plasma membrane [GO:1900930] (BP) Also known as: negative regulation of L-tyrosine import, down regulation of L-tyrosine import, down-regulation of L-tyrosine import, downregulation of L-tyrosine import, inhibition of L-tyrosine import, down regulation of L-tyrosine uptake, down-regulation of L-tyrosine uptake, downregulation of L-tyrosine uptake, inhibition of L-tyrosine uptake, negative regulation of L-tyrosine uptake Sources: GOC:TermGenie Definition: Any process that stops, prevents or reduces the frequency, rate or extent of L-tyrosine import into the cell. Relationships: is a type of negative regulation of organic acid transport [GO:0032891]; is a type of negative regulation of transmembrane transport [GO:0034763]; is a type of GO:0051956; is a type of regulation of L-tyrosine import across plasma membrane [GO:1900929]; negatively regulates GO:1903808